{
  "gene_name": "Putative uncharacterized protein UNQ5830_PRO19650_PRO19816",
  "term_id": "GO:0043123",
  "gene_symbol": "UNQ5830/PRO19650/PRO19816",
  "gene": "UniProtKB:Q6UY13",
  "term_label": "positive regulation of canonical NF-kappaB signal transduction"
}